{
  "gene_symbol": "GRIK5",
  "gene": "UniProtKB:Q16478",
  "gene_name": "Glutamate receptor ionotropic, kainate 5",
  "term_label": "kainate selective glutamate receptor complex",
  "term_id": "GO:0032983"
}